{
  "gene": "UniProtKB:Q9BQI3",
  "gene_symbol": "EIF2AK1",
  "term_label": "eukaryotic translation initiation factor 2alpha kinase activity",
  "term_id": "GO:0004694",
  "gene_name": "Eukaryotic translation initiation factor 2-alpha kinase 1"
}